cerebellum development [GO:0021549] (biological process) Sources: GOC:cls, GOC:dgh, GOC:dph, GOC:jid, GO_REF:0000021 Relationships: is_a anatomical structure development [GO:0048856]; is part of metencephalon development [GO:0022037] Definition: The process whose specific outcome is the progression of the cerebellum over time, from its formation to the mature structure. The cerebellum is the portion of the brain in the back of the head between the cerebrum and the pons. In mice, the cerebellum controls balance for walking and standing, modulates the force and range of movement and is involved in the learning of motor skills.